{
  "term_label": "electron transport coupled proton transport",
  "gene": "UniProtKB:P03915",
  "gene_name": "NADH-ubiquinone oxidoreductase chain 5",
  "term_id": "GO:0015990",
  "gene_symbol": "MT-ND5"
}